cardioblast migration to the midline involved in heart rudiment formation [GO:0003319] (biological process) Relationships: is a type of GO:0003318; is part of heart rudiment formation [GO:0003315] Definition: The orderly movement of a cardioblast toward the midline that contributes to the initial appearance of the heart rudiment. Sources: GOC:mtg_heart